{
  "gene_symbol": "FNTA",
  "gene_name": "Protein farnesyltransferase_geranylgeranyltransferase type-1 subunit alpha",
  "term_label": "cytoplasm",
  "gene": "UniProtKB:P49354",
  "term_id": "GO:0005737"
}